B1 bradykinin receptor binding [GO:0031712] (molecular function) Definition: Binding to a B1 bradykinin receptor. Also known as: B1 bradykinin receptor ligand Sources: GOC:mah, GOC:nln Relationships: is a type of GO:0031711